{
  "gene_symbol": "TIAM1",
  "gene_name": "Rho guanine nucleotide exchange factor TIAM1",
  "gene": "UniProtKB:Q13009",
  "term_id": "GO:0005886",
  "term_label": "plasma membrane"
}